UDP-glucuronate transmembrane transporter activity [GO:0005461] (molecular function) Definition: Enables the transfer of a UDP-glucuronic acid from one side of a membrane to the other. UDP-glucuronic acid is a substance composed of glucuronic acid in glycosidic linkage with uridine diphosphate. Sources: GOC:ai, GOC:mtg_transport, ISBN:0815340729 Also known as: UDP-glucuronic acid transmembrane transporter activity Relationships: is_a pyrimidine nucleotide-sugar transmembrane transporter activity [GO:0015165]; is a type of carboxylic acid transmembrane transporter activity [GO:0046943]; is part of UDP-glucuronate transmembrane transport [GO:0015787]